{
  "term_id": "GO:0061891",
  "gene": "UniProtKB:Q9H2B2",
  "term_label": "calcium ion sensor activity",
  "gene_symbol": "SYT4",
  "gene_name": "Synaptotagmin-4"
}